positive regulation of synaptic plasticity by chemical substance [GO:0051914] (biological process) Subtypes: induction of synaptic plasticity by chemical substance [GO:0051915] Definition: The process in which a chemical substance increases synaptic plasticity, the ability of synapses to change as circumstances require. Also known as: up regulation of synaptic plasticity by chemical substance, up-regulation of synaptic plasticity by chemical substance, upregulation of synaptic plasticity by chemical substance, activation of synaptic plasticity by chemical substance, positive regulation of synaptic plasticity by drug, stimulation of synaptic plasticity by chemical substance Sources: GOC:ai Relationships: is a type of GO:0031915; is a type of regulation of synaptic plasticity by chemical substance [GO:0051913]